{
  "gene_name": "Zinc finger protein 275",
  "gene_symbol": "ZNF275",
  "term_id": "UNKNOWN:0003",
  "gene": "UniProtKB:Q9NSD4",
  "term_label": "Unknown cellular component"
}